chemokine (C-C motif) ligand 21 production [GO:0097389] (biological process) Definition: The appearance of chemokine (C-C motif) ligand 21 (CCL21) due to biosynthesis or secretion following a cellular stimulus, resulting in an increase in its intracellular or extracellular levels. Sources: GOC:rv Also known as: CCL21 production Relationships: is_a GO:0032602